{
  "term_label": "induction of positive chemotaxis",
  "term_id": "GO:0050930",
  "gene": "UniProtKB:P15692",
  "gene_symbol": "VEGFA",
  "gene_name": "Vascular endothelial growth factor A, long form"
}